telomere maintenance via recombination [GO:0000722] (biological process) Regulation: regulated by GO:0032207; negatively regulated by negative regulation of telomere maintenance via recombination [GO:0032208]; positively regulated by positive regulation of telomere maintenance via recombination [GO:0032209] Definition: Any recombinational process that contributes to the maintenance of proper telomeric length. Relationships: is a type of telomere maintenance [GO:0000723]; is a type of mitotic recombination [GO:0006312] References: PMID:11850777 Sources: GOC:elh Also known as: telomerase-independent telomere maintenance Subtypes: telomeric DNA-containing double minutes formation [GO:0061819]